{
  "gene_symbol": "SQOR",
  "term_label": "sulfide oxidation, using sulfide:quinone oxidoreductase",
  "term_id": "GO:0070221",
  "gene_name": "Sulfide:quinone oxidoreductase, mitochondrial",
  "gene": "UniProtKB:Q9Y6N5"
}